{
  "term_id": "GO:0010468",
  "term_label": "regulation of gene expression",
  "gene_name": "PR domain zinc finger protein 13",
  "gene": "UniProtKB:Q9H4Q3",
  "gene_symbol": "PRDM13"
}